{
  "gene_symbol": "FRMD4A",
  "term_label": "Unknown biological process",
  "gene_name": "FERM domain-containing protein 4A",
  "term_id": "UNKNOWN:0002",
  "gene": "UniProtKB:Q9P2Q2"
}